{
  "gene": "UniProtKB:Q6ZSC3",
  "gene_symbol": "RBM43",
  "gene_name": "RNA-binding protein 43",
  "term_id": "UNKNOWN:0003",
  "term_label": "Unknown cellular component"
}